{
  "gene": "UniProtKB:Q96AE7",
  "term_label": "actin filament polymerization",
  "gene_name": "Tetratricopeptide repeat protein 17",
  "term_id": "GO:0030041",
  "gene_symbol": "TTC17"
}